methylenetetrahydrofolate reductase (NADPH) activity [GO:0106313] (MF) Relationships: is a type of methylenetetrahydrofolate reductase [NAD(P)H] activity [GO:0004489] Definition: Catalysis of the reaction: (6S)-5-methyl-5,6,7,8-tetrahydrofolate + NADP+ = (6R)-5,10-methylene-5,6,7,8-tetrahydrofolate + NADPH + H+. Sources: RHEA:19817